{
  "gene_symbol": "GMPPA",
  "gene": "UniProtKB:Q96IJ6",
  "gene_name": "Mannose-1-phosphate guanyltransferase alpha",
  "term_id": "GO:0005737",
  "term_label": "cytoplasm"
}